{
  "term_label": "Unknown molecular function",
  "gene": "UniProtKB:Q8N7B1",
  "gene_symbol": "HORMAD2",
  "gene_name": "HORMA domain-containing protein 2",
  "term_id": "UNKNOWN:0001"
}